{
  "term_id": "GO:0004984",
  "gene_name": "Putative olfactory receptor 8G3 pseudogene",
  "gene_symbol": "OR8G3",
  "term_label": "olfactory receptor activity",
  "gene": "UniProtKB:P0DMU2"
}